{
  "term_id": "GO:0080008",
  "gene_name": "DDB1- and CUL4-associated factor 6",
  "gene": "UniProtKB:Q58WW2",
  "gene_symbol": "DCAF6",
  "term_label": "Cul4-RING E3 ubiquitin ligase complex"
}